{
  "gene": "UniProtKB:P48739",
  "term_label": "Unknown biological process",
  "gene_symbol": "PITPNB",
  "gene_name": "Phosphatidylinositol transfer protein beta isoform",
  "term_id": "UNKNOWN:0002"
}